{
  "gene_name": "Dual specificity protein phosphatase 22",
  "term_label": "cytosol",
  "gene_symbol": "DUSP22",
  "gene": "UniProtKB:Q9NRW4",
  "term_id": "GO:0005829"
}